{
  "gene": "UniProtKB:Q63ZE4",
  "gene_name": "Solute carrier family 22 member 10",
  "gene_symbol": "SLC22A10",
  "term_label": "Unknown cellular component",
  "term_id": "UNKNOWN:0003"
}